{
  "gene_name": "3-oxo-5-alpha-steroid 4-dehydrogenase 1",
  "term_label": "neuronal cell body",
  "term_id": "GO:0043025",
  "gene_symbol": "SRD5A1",
  "gene": "UniProtKB:P18405"
}